{
  "term_label": "cell-cell junction",
  "gene_name": "Transforming growth factor beta-1-induced transcript 1 protein",
  "term_id": "GO:0005911",
  "gene_symbol": "TGFB1I1",
  "gene": "UniProtKB:O43294"
}